gallate catabolic process [GO:0019396] (biological process) Subtypes: anaerobic gallate catabolic process [GO:0019328], aerobic gallate catabolic process [GO:0042195] Also known as: gallate breakdown, gallate catabolism, gallate degradation, gallic acid catabolic process, gallic acid catabolism, gallate metabolic process, gallate metabolism, gallic acid metabolic process, gallic acid metabolism Sources: GOC:jl Relationships: is a type of phenol-containing compound catabolic process [GO:0019336]; is a type of benzene-containing compound metabolic process [GO:0042537]; is a type of monocarboxylic acid catabolic process [GO:0072329] Definition: The chemical reactions and pathways resulting in the breakdown of gallate, the anion of gallic acid (3,4,5-trihydroxybenzoic acid).